{
  "gene_name": "Serine_threonine-protein kinase H1",
  "term_label": "protein serine/threonine kinase activity",
  "term_id": "GO:0004674",
  "gene_symbol": "PSKH1",
  "gene": "UniProtKB:P11801"
}